{
  "gene_name": "Ankyrin repeat and sterile alpha motif domain-containing protein 1B",
  "gene": "UniProtKB:Q7Z6G8",
  "term_id": "GO:0098978",
  "term_label": "glutamatergic synapse",
  "gene_symbol": "ANKS1B"
}